retroviral 3' processing activity [GO:0044824] (molecular function) Definition: The catalysis of the removal of two di- or tri-nucleotides from each 3' end of double-stranded viral DNA, exposing recessed 3' hydroxyls. Relationships: is a type of DNA endonuclease activity [GO:0004520]; is a type of hydrolase activity, acting on ester bonds [GO:0016788]; is part of retroviral integrase activity [GO:0044823] References: PMID:22580823 Note: This reaction may serve to remove heterogeneous extra bases from the viral DNA end, and to stabilize the integrase-DNA complex. The chemistry of cleavage is a simple hydrolysis by single-step transesterification. Also known as: 3' processing reaction, 3'-processing activity